L-leucine metabolic process [GO:0006551] (biological process) Definition: The chemical reactions and pathways involving L-leucine, 2-amino-4-methylpentanoic acid. Relationships: is_a branched-chain amino acid metabolic process [GO:0009081]; is_a L-amino acid metabolic process [GO:0170033]; is a type of proteinogenic amino acid metabolic process [GO:0170039] Also known as: leucine metabolic process, L-leucine metabolism Sources: GOC:ai Subtypes: GO:0006552, L-leucine biosynthetic process [GO:0009098]